{
  "gene": "UniProtKB:Q8WW18",
  "term_label": "Unknown molecular function",
  "gene_name": "Uncharacterized protein C17orf50",
  "term_id": "UNKNOWN:0001",
  "gene_symbol": "C17orf50"
}